{
  "gene_symbol": "PABPC5",
  "gene_name": "Polyadenylate-binding protein 5",
  "term_id": "GO:0008143",
  "term_label": "poly(A) binding",
  "gene": "UniProtKB:Q96DU9"
}